{
  "gene": "UniProtKB:P20336",
  "gene_name": "Ras-related protein Rab-3A",
  "term_id": "GO:0031489",
  "gene_symbol": "RAB3A",
  "term_label": "myosin V binding"
}